glycosylphosphatidylinositol diacylglycerol-lyase activity [GO:0047396] (molecular function) Relationships: is a type of phosphorus-oxygen lyase activity [GO:0016849] Definition: Catalysis of the reaction: 6-(alpha-D-glucosaminyl)-1-phosphatidyl-1D-myo-inositol = 1,2-diacyl-sn-glycerol + 6-(alpha-D-glucosaminyl)-1D-myo-inositol 1,2-cyclic phosphate. Sources: EC:4.6.1.14, MetaCyc:3.1.4.47-RXN Also known as: variant-surface-glycoprotein phospholipase C activity, glycosylphosphatidylinositol-phospholipase C activity, (glycosyl)phosphatidylinositol-specific phospholipase C activity, 6-(alpha-D-glucosaminyl)-1-phosphatidyl-1D-myo-inositol diacyl-sn-glycerol-lyase [6-(alpha-D-glucosaminyl)-1D-myo-inositol 1,2-cyclic phosphate-forming], 6-(alpha-D-glucosaminyl)-1-phosphatidyl-1D-myo-inositol diacylglycerol-lyase (1,2-cyclic-phosphate-forming) activity, GPI-PLC activity, GPI-specific phospholipase C activity, VSG-lipase activity, glycosyl inositol phospholipid anchor-hydrolyzing enzyme activity, glycosylphosphatidylinositol-specific phospholipase C activity